{
  "gene_symbol": "ULK2",
  "gene": "UniProtKB:Q8IYT8",
  "gene_name": "Serine_threonine-protein kinase ULK2",
  "term_id": "GO:0048671",
  "term_label": "negative regulation of collateral sprouting"
}